positive regulation of vascular associated smooth muscle cell differentiation [GO:1905065] (biological process) Definition: Any process that activates or increases the frequency, rate or extent of vascular smooth muscle cell differentiation. References: PMID:19088079 Sources: GOC:BHF, GOC:BHF_miRNA, GOC:TermGenie, GOC:rph, GO_REF:0000058 Also known as: positive regulation of VSMC differentiation, positive regulation of vascular smooth muscle cell differentiation, up regulation of VSMC differentiation, up regulation of vascular associated smooth muscle cell differentiation, up regulation of vascular smooth muscle cell differentiation, up-regulation of VSMC differentiation, up-regulation of vascular associated smooth muscle cell differentiation, up-regulation of vascular smooth muscle cell differentiation, upregulation of VSMC differentiation, upregulation of vascular associated smooth muscle cell differentiation, upregulation of vascular smooth muscle cell differentiation, activation of VSMC differentiation, activation of vascular associated smooth muscle cell differentiation, activation of vascular smooth muscle cell differentiation Relationships: is a type of GO:0051152; is a type of regulation of vascular associated smooth muscle cell differentiation [GO:1905063]; positively regulates vascular associated smooth muscle cell differentiation [GO:0035886] Subtypes: positive regulation of aortic smooth muscle cell differentiation [GO:1904831], positive regulation of vascular associated smooth muscle cell differentiation involved in phenotypic switching [GO:1905932], positive regulation of cardiac vascular smooth muscle cell differentiation [GO:2000724]